{
  "gene": "UniProtKB:P46937",
  "term_id": "GO:0045944",
  "term_label": "positive regulation of transcription by RNA polymerase II",
  "gene_symbol": "YAP1",
  "gene_name": "Transcriptional coactivator YAP1"
}